regulation of otic vesicle morphogenesis [GO:1904118] (biological process) Relationships: is a type of regulation of morphogenesis of an epithelium [GO:1905330]; is a type of regulation of animal organ morphogenesis [GO:2000027]; regulates otic vesicle morphogenesis [GO:0071600] References: PMID:25677106 Sources: GOC:TermGenie, GO_REF:0000058 Definition: Any process that modulates the frequency, rate or extent of otic vesicle morphogenesis. Subtypes: negative regulation of otic vesicle morphogenesis [GO:1904119], positive regulation of otic vesicle morphogenesis [GO:1904120]